{
  "gene_name": "ATP-dependent RNA helicase DDX19A",
  "gene": "UniProtKB:Q9NUU7",
  "gene_symbol": "DDX19A",
  "term_label": "nucleus",
  "term_id": "GO:0005634"
}